{
  "term_id": "GO:0051601",
  "gene": "UniProtKB:Q17RC7",
  "term_label": "exocyst localization",
  "gene_name": "Exocyst complex component 3-like protein 4",
  "gene_symbol": "EXOC3L4"
}